{
  "gene": "UniProtKB:P48169",
  "term_label": "synaptic transmission, GABAergic",
  "term_id": "GO:0051932",
  "gene_name": "Gamma-aminobutyric acid receptor subunit alpha-4",
  "gene_symbol": "GABRA4"
}